{
  "term_label": "positive regulation of synapse assembly",
  "gene_name": "Amphoterin-induced protein 2",
  "gene_symbol": "AMIGO2",
  "term_id": "GO:0051965",
  "gene": "UniProtKB:Q86SJ2"
}